establishment of protein localization to mitochondrion [GO:0072655] (BP) Relationships: is a type of establishment of protein localization to organelle [GO:0072594] Definition: The directed movement of a protein to the mitochondrion or a part of the mitochondrion. Also known as: establishment of protein localisation to mitochondrion, establishment of protein localization in mitochondrion Sources: GOC:mah Subtypes: protein targeting to mitochondrion [GO:0006626], protein import into mitochondrial matrix [GO:0030150], protein import into mitochondrial intermembrane space [GO:0045041], establishment of protein localization to mitochondrial membrane [GO:0090151] Regulation: regulated by regulation of establishment of protein localization to mitochondrion [GO:1903747]; negatively regulated by negative regulation of establishment of protein localization to mitochondrion [GO:1903748]; positively regulated by positive regulation of establishment of protein localization to mitochondrion [GO:1903749]